{
  "term_label": "cytosol",
  "gene_symbol": "NFKBIA",
  "gene_name": "NF-kappa-B inhibitor alpha",
  "term_id": "GO:0005829",
  "gene": "UniProtKB:P25963"
}